positive regulation of unsaturated fatty acid biosynthetic process [GO:2001280] (biological process) Subtypes: GO:0031394 Definition: Any process that activates or increases the frequency, rate or extent of unsaturated fatty acid biosynthetic process. Also known as: positive regulation of unsaturated fatty acid anabolism, positive regulation of unsaturated fatty acid biosynthesis, positive regulation of unsaturated fatty acid formation, positive regulation of unsaturated fatty acid synthesis, positive regulation of fatty acid desaturation, positive regulation of polyunsaturated fatty acid biosynthesis Sources: GO:0006636 Relationships: is a type of positive regulation of fatty acid biosynthetic process [GO:0045723]; is_a GO:2001279; positively regulates unsaturated fatty acid biosynthetic process [GO:0006636]